{
  "gene_name": "CDGSH iron-sulfur domain-containing protein 2",
  "gene": "UniProtKB:Q8N5K1",
  "term_label": "2 iron, 2 sulfur cluster binding",
  "term_id": "GO:0051537",
  "gene_symbol": "CISD2"
}